xylan metabolic process [GO:0045491] (biological process) Definition: The chemical reactions and pathways involving xylan, a polymer containing a beta-1,4-linked D-xylose backbone. Also known as: xylan metabolism References: PMID:11931668 Sources: GOC:go_curators Subtypes: glucuronoxylan metabolic process [GO:0010413], GO:0045492, xylan catabolic process [GO:0045493] Relationships: is a type of polysaccharide metabolic process [GO:0005976]